{
  "gene_symbol": "TBC1D3G",
  "term_id": "UNKNOWN:0002",
  "term_label": "Unknown biological process",
  "gene_name": "TBC1 domain family member 3G",
  "gene": "UniProtKB:Q6DHY5"
}